{
  "gene": "UniProtKB:Q9H2X6",
  "gene_name": "Homeodomain-interacting protein kinase 2",
  "gene_symbol": "HIPK2",
  "term_label": "SMAD binding",
  "term_id": "GO:0046332"
}